intracellular oxygen homeostasis [GO:0032364] (biological process) Also known as: oxygen homeostasis, cellular oxygen homeostasis Sources: GOC:rph Relationships: is a type of intracellular chemical homeostasis [GO:0055082] Definition: A homeostatic process involved in the maintenance of a steady state level of oxygen within a cell.